{
  "gene_symbol": "IFT70A",
  "gene_name": "Intraflagellar transport protein 70A",
  "term_id": "GO:0042073",
  "term_label": "intraciliary transport",
  "gene": "UniProtKB:Q86WT1"
}